regulation of execution phase of apoptosis [GO:1900117] (biological process) Sources: GOC:TermGenie, GOC:mtg_apoptosis Definition: Any process that modulates the frequency, rate or extent of execution phase of apoptosis. Relationships: is a type of GO:0050794; regulates execution phase of apoptosis [GO:0097194] Subtypes: negative regulation of execution phase of apoptosis [GO:1900118], positive regulation of execution phase of apoptosis [GO:1900119]